{
  "gene": "UniProtKB:O75602",
  "gene_symbol": "SPAG6",
  "gene_name": "Sperm-associated antigen 6",
  "term_label": "neuron projection extension",
  "term_id": "GO:1990138"
}